{
  "gene": "UniProtKB:P61599",
  "gene_symbol": "NAA20",
  "term_label": "regulation of actin cytoskeleton organization",
  "term_id": "GO:0032956",
  "gene_name": "N-alpha-acetyltransferase 20"
}